{
  "gene_name": "Nucleophosmin",
  "gene_symbol": "NPM1",
  "gene": "UniProtKB:P06748",
  "term_label": "RNA binding",
  "term_id": "GO:0003723"
}